{
  "term_label": "regulation of synaptic assembly at neuromuscular junction",
  "term_id": "GO:0008582",
  "gene_name": "Protein lin-7 homolog B",
  "gene": "UniProtKB:Q9HAP6",
  "gene_symbol": "LIN7B"
}